tRNA gene clustering [GO:0070058] (biological process) Definition: The process in which tRNA genes, which are not linearly connected on the chromosome, are transported in three dimensions to, and maintained together in, the nucleolus. This clustered positioning leads to transcriptional silencing of nearby RNA polymerase II promoters (termed tRNA gene mediated (tgm) silencing) in S. cerevisiae. Relationships: is a type of chromosome organization [GO:0051276] References: PMID:18708579 Sources: GOC:jh, GOC:mah